forebrain astrocyte differentiation [GO:0021896] (biological process) References: PMID:16226447 Sources: GOC:cls, GOC:dgh, GOC:dph, GOC:jid, GO_REF:0000021 Definition: The process in which a relatively unspecialized cell acquires the specialized features of an astrocyte residing in the forebrain. An astrocyte is the most abundant type of glial cell. Astrocytes provide support for neurons and regulate the environment in which they function. Relationships: is a type of astrocyte differentiation [GO:0048708]; is part of forebrain development [GO:0030900]